{
  "gene_name": "Transmembrane protein 250",
  "term_id": "UNKNOWN:0002",
  "term_label": "Unknown biological process",
  "gene_symbol": "TMEM250",
  "gene": "UniProtKB:H0YL14"
}